structural constituent of cytoplasmic lattice [GO:0140094] (molecular function) Relationships: is a type of GO:0005198 References: PMID:37922900 Definition: The action of a molecule that contributes to the structural integrity of cytoplasmic lattice of the the mammalian ooplasm.